{
  "gene_name": "Lysosomal Pro-X carboxypeptidase",
  "term_label": "angiogenesis involved in wound healing",
  "gene": "UniProtKB:P42785",
  "gene_symbol": "PRCP",
  "term_id": "GO:0060055"
}